endothelin receptor signaling pathway involved in heart process [GO:0086101] (biological process) References: PMID:17376402 Sources: GOC:BHF, GOC:mtg_cardiac_conduct_nov11 Also known as: endothelin receptor signalling pathway involved in heart process Relationships: is a type of GO:0086100; is a type of G protein-coupled receptor signaling pathway involved in heart process [GO:0086103] Definition: An endothelin receptor signaling pathway which contributes to a circulatory system process carried out by the heart.